{
  "gene_name": "snRNA-activating protein complex subunit 2",
  "term_label": "Unknown biological process",
  "gene_symbol": "SNAPC2",
  "gene": "UniProtKB:Q13487",
  "term_id": "UNKNOWN:0002"
}